L-lysine transmembrane export from vacuole [GO:0089707] (biological process) Definition: The directed movement of L-lysine out of the vacuole, across the vacuolar membrane. References: PMID:21307582 Relationships: is a type of GO:0032974; is a type of L-lysine transmembrane transport [GO:1903401] Subtypes: L-lysine transmembrane transport from lysosomal lumen to cytosol [GO:1904916]